linoleate 11-lipoxygenase activity [GO:0050584] (molecular function) Definition: Catalysis of the reaction: linoleate + O2 = (9Z,11S,12Z)-11-hydroperoxyoctadeca-9,12-dienoate. Sources: EC:1.13.11.45, RHEA:18993 Also known as: linoleate dioxygenase activity, linoleate:oxygen 11S-oxidoreductase activity, manganese lipoxygenase activity Relationships: is a type of oxidoreductase activity, acting on single donors with incorporation of molecular oxygen, incorporation of two atoms of oxygen [GO:0016702]